interkinetic nuclear migration [GO:0022027] (biological process) Relationships: is a type of nuclear migration [GO:0007097]; is part of GO:0021846 Sources: GOC:cls, GOC:dgh, GOC:dph, GOC:jid, GO_REF:0000021 Definition: The movement of the nucleus of the ventricular zone cell between the apical and the basal zone surfaces. Mitosis occurs when the nucleus is near the apical surface, that is, the lumen of the ventricle.